{
  "gene": "UniProtKB:Q9NS82",
  "gene_name": "Asc-type amino acid transporter 1",
  "term_id": "GO:0015175",
  "term_label": "neutral L-amino acid transmembrane transporter activity",
  "gene_symbol": "SLC7A10"
}